{
  "term_id": "GO:0004032",
  "term_label": "aldose reductase (NADPH) activity",
  "gene_name": "Aldo-keto reductase family 1 member C2",
  "gene": "UniProtKB:P52895",
  "gene_symbol": "AKR1C2"
}